mitotic nuclear membrane disassembly [GO:0007077] (BP) References: PMID:32848252 Sources: GOC:bf Regulation: regulated by regulation of mitotic nuclear envelope disassembly [GO:1905557]; negatively regulated by negative regulation of mitotic nuclear envelope disassembly [GO:1905558]; positively regulated by positive regulation of mitotic nuclear envelope disassembly [GO:1905559] Also known as: NEB, local NEB, nuclear envelope breakdown, mitotic nuclear envelope breakdown, mitotic nuclear envelope catabolism, mitotic nuclear envelope degradation, mitotic nuclear envelope disassembly Subtypes: mitotic nuclear pore complex disassembly [GO:0140516] Relationships: is a type of nuclear membrane disassembly [GO:0051081]; is a type of mitotic cell cycle process [GO:1903047] Definition: The mitotic cell cycle process in which the controlled partial or complete breakdown of the nuclear membranes during occurs during mitosis.